{
  "term_id": "GO:0005794",
  "term_label": "Golgi apparatus",
  "gene_symbol": "CEPT1",
  "gene": "UniProtKB:Q9Y6K0",
  "gene_name": "Choline_ethanolaminephosphotransferase 1"
}